{
  "gene_name": "Haloacid dehalogenase-like hydrolase domain-containing protein 3",
  "term_label": "Unknown biological process",
  "term_id": "UNKNOWN:0002",
  "gene": "UniProtKB:Q9BSH5",
  "gene_symbol": "HDHD3"
}